{
  "gene_symbol": "SAMD4A",
  "gene": "UniProtKB:Q9UPU9",
  "term_id": "GO:0003729",
  "term_label": "mRNA binding",
  "gene_name": "Protein Smaug homolog 1"
}